{
  "gene": "UniProtKB:P43628",
  "term_id": "GO:0004888",
  "term_label": "transmembrane signaling receptor activity",
  "gene_name": "Killer cell immunoglobulin-like receptor 2DL3",
  "gene_symbol": "KIR2DL3"
}